{
  "term_label": "Unknown cellular component",
  "gene": "UniProtKB:Q9NRM2",
  "gene_name": "Zinc finger protein 277",
  "gene_symbol": "ZNF277",
  "term_id": "UNKNOWN:0003"
}